{
  "gene_name": "Solute carrier family 52, riboflavin transporter, member 2",
  "term_id": "GO:0032218",
  "term_label": "riboflavin transport",
  "gene_symbol": "SLC52A2",
  "gene": "UniProtKB:Q9HAB3"
}